{
  "term_label": "guanyl-nucleotide exchange factor activity",
  "term_id": "GO:0005085",
  "gene_symbol": "ALS2",
  "gene_name": "Alsin",
  "gene": "UniProtKB:Q96Q42"
}